{
  "gene": "UniProtKB:Q9NZP6",
  "gene_symbol": "NPAP1",
  "term_id": "GO:0008139",
  "gene_name": "Nuclear pore-associated protein 1",
  "term_label": "nuclear localization sequence binding"
}